{
  "gene_symbol": "DIP2C-AS1",
  "term_id": "UNKNOWN:0002",
  "gene_name": "Putative uncharacterized protein DIP2C-AS1",
  "term_label": "Unknown biological process",
  "gene": "UniProtKB:Q8N8Z3"
}